RNA stem-loop binding [GO:0035613] (molecular function) References: PMID:16568238, PMID:20455544 Sources: GOC:sart Relationships: is a type of RNA binding [GO:0003723] Subtypes: snRNA stem-loop binding [GO:0035614] Also known as: RNA hairpin binding, RNA hairpin loop binding Definition: Binding to a stem-loop in an RNA molecule. An RNA stem-loop is a secondary RNA structure consisting of a double-stranded RNA (dsRNA) stem and a terminal loop.